{
  "term_label": "purine nucleoside metabolic process",
  "gene": "UniProtKB:Q9BQ69",
  "gene_name": "ADP-ribose glycohydrolase MACROD1",
  "gene_symbol": "MACROD1",
  "term_id": "GO:0042278"
}